{
  "gene": "UniProtKB:Q96K30",
  "term_label": "nuclear export",
  "term_id": "GO:0051168",
  "gene_symbol": "RITA1",
  "gene_name": "RBPJ-interacting and tubulin-associated protein 1"
}